calcium ion import into cytosol [GO:1902656] (biological process) Relationships: is a type of GO:0006816 Subtypes: GO:0098703 Definition: The directed movement of calcium ion into a cytosol. Also known as: calcium import into cytosol Sources: GOC:TermGenie, GOC:vw, GO_REF:0000075